helper T cell extravasation [GO:0035684] (biological process) Relationships: is a type of T cell extravasation [GO:0072683] Definition: The migration of a helper T cell from the blood vessels into the surrounding tissue. A helper T-cell is an effector T cell that provides help in the form of secreted cytokines to other immune cells. Also known as: T-helper cell extravasation, helper T-cell extravasation Subtypes: T-helper 1 cell extravasation [GO:0035687], T-helper 17 cell extravasation [GO:0035699] Sources: CL:0000912, GOC:BHF